{
  "gene_name": "Tensin-1",
  "gene_symbol": "TNS1",
  "gene": "UniProtKB:Q9HBL0",
  "term_label": "fibroblast migration",
  "term_id": "GO:0010761"
}